{
  "term_label": "vesicle-mediated transport",
  "gene_name": "F-box only protein 8",
  "term_id": "GO:0016192",
  "gene": "UniProtKB:Q9NRD0",
  "gene_symbol": "FBXO8"
}